{
  "term_label": "neuron projection development",
  "gene_name": "Receptor-type tyrosine-protein phosphatase mu",
  "gene_symbol": "PTPRM",
  "term_id": "GO:0031175",
  "gene": "UniProtKB:P28827"
}